{
  "gene_name": "Solute carrier family 35 member F3",
  "gene": "UniProtKB:Q8IY50",
  "term_id": "GO:0015888",
  "term_label": "thiamine transport",
  "gene_symbol": "SLC35F3"
}